{
  "gene_symbol": "YPEL2",
  "gene_name": "Protein yippee-like 2",
  "gene": "UniProtKB:Q96QA6",
  "term_label": "Unknown molecular function",
  "term_id": "UNKNOWN:0001"
}